mycothione reductase [NAD(P)H] activity [GO:0050627] (molecular function) Relationships: is a type of oxidoreductase activity, acting on a sulfur group of donors, NAD(P) as acceptor [GO:0016668] Sources: EC:1.8.1.15 Also known as: mycothiol-disulfide reductase activity, mycothiol:NAD(P)+ oxidoreductase activity Definition: Catalysis of the reaction: NAD(P)+ + mycothiol = NAD(P)H + H+ + mycothione.